{
  "gene": "UniProtKB:Q8N6N3",
  "term_id": "UNKNOWN:0003",
  "gene_name": "UPF0690 protein C1orf52",
  "term_label": "Unknown cellular component",
  "gene_symbol": "C1orf52"
}